{
  "gene": "UniProtKB:Q9Y4G8",
  "term_id": "GO:0005886",
  "gene_symbol": "RAPGEF2",
  "term_label": "plasma membrane",
  "gene_name": "Rap guanine nucleotide exchange factor 2"
}